{
  "gene_symbol": "ADH5",
  "gene_name": "Alcohol dehydrogenase class-3",
  "gene": "UniProtKB:P11766",
  "term_id": "GO:0046294",
  "term_label": "formaldehyde catabolic process"
}